{
  "term_id": "GO:0034039",
  "gene": "UniProtKB:Q9UIF7",
  "gene_symbol": "MUTYH",
  "term_label": "8-oxo-7,8-dihydroguanine DNA N-glycosylase activity",
  "gene_name": "Adenine DNA glycosylase"
}